{
  "gene_name": "Neuropeptide B",
  "term_id": "GO:0007631",
  "term_label": "feeding behavior",
  "gene": "UniProtKB:Q8NG41",
  "gene_symbol": "NPB"
}